{
  "term_id": "GO:0005544",
  "term_label": "calcium-dependent phospholipid binding",
  "gene_name": "Cytosolic phospholipase A2 gamma",
  "gene": "UniProtKB:Q9UP65",
  "gene_symbol": "PLA2G4C"
}